cardiolipin synthase activity [GO:0008808] (molecular function) Relationships: is a type of phosphatidyltransferase activity [GO:0030572] Also known as: cardiolipin synthetase activity, diphosphatidylglycerol synthase activity, cardiolipin synthase 2 activity, cardiolipin synthetase 2 activity Sources: GOC:jl, RHEA:31451 Definition: Catalysis of the reaction: phosphatidylglycerol + phosphatidylglycerol = diphosphatidylglycerol (cardiolipin) + glycerol.